acetylgalactosaminyl-O-glycosyl-glycoprotein beta-1,3-N-acetylglucosaminyltransferase activity [GO:0047224] (molecular function) Definition: Catalysis of the reaction: 3-O-N-acetyl-D-galactosalaminyl-[protein] + UDP-N-acetyl-D-glucosamine = 3-O-N-acetyl-beta-D-glucosaminyl-1,3-N-acetyl-D-galactosaminyl-[protein] + UDP. Linkage of the glycan to the protein occurs via the oxygen atom in the side chain of an L-serine or L-threonine residue. Sources: EC:2.4.1.147 Also known as: O-glycosyl-oligosaccharide-glycoprotein N-acetylglucosaminyltransferase III activity, UDP-N-acetyl-D-glucosamine:O-glycosyl-glycoprotein (N-acetyl-D-glucosamine to N-acetyl-D-galactosaminyl-R) beta-1,3-N-acetyl-D-glucosaminyltransferase activity, core 3-beta-GlcNAc-transferase activity, core 3beta-GlcNAc-transferase activity, mucin core 3 beta3-GlcNAc-transferase activity, uridine diphosphoacetylglucosamine-mucin beta(1->3)-acetylglucosaminyltransferase activity Relationships: is a type of acetylglucosaminyltransferase activity [GO:0008375]; is a type of GO:0140103